{
  "gene": "UniProtKB:P0C646",
  "gene_name": "Olfactory receptor 52Z1P",
  "term_id": "UNKNOWN:0002",
  "gene_symbol": "OR52Z1P",
  "term_label": "Unknown biological process"
}